{
  "gene": "UniProtKB:Q8WTX9",
  "term_id": "GO:0006612",
  "gene_symbol": "ZDHHC1",
  "term_label": "protein targeting to membrane",
  "gene_name": "Palmitoyltransferase ZDHHC1"
}